{
  "gene_symbol": "ASZ1",
  "term_label": "Unknown biological process",
  "gene": "UniProtKB:Q8WWH4",
  "term_id": "UNKNOWN:0002",
  "gene_name": "Ankyrin repeat, SAM and basic leucine zipper domain-containing protein 1"
}